xenobiotic catabolic process [GO:0042178] (biological process) Definition: The chemical reactions and pathways resulting in the breakdown of a xenobiotic compound, a compound foreign to the organism exposed to it, carried out by individual cells. It may be synthesized by another organism (like ampicilin) or it can be a synthetic chemical. Sources: GOC:jl, GOC:krc Relationships: is a type of xenobiotic metabolic process [GO:0006805]; is_a catabolic process [GO:0009056] Subtypes: phenylacetate catabolic process [GO:0010124], anaerobic cyclohexane-1-carboxylate catabolic process [GO:0010129], dibenzothiophene catabolic process [GO:0018896], GO:0018897, GO:0019256, adamantanone catabolic process [GO:0019263], methylquinoline catabolic process [GO:0019335], dibenzofuran catabolic process [GO:0019340], dibenzo-p-dioxin catabolic process [GO:0019341], 3-phenylpropionate catabolic process [GO:0019380], caprolactam catabolic process [GO:0019384], cyclohexanol oxidation [GO:0019399], GO:0019429, GO:0019487, n-octane oxidation [GO:0019498], GO:0019501, phenylmercury acetate catabolic process [GO:0019506], GO:0019610, 6-hydroxycineole catabolic process [GO:0019639], nylon catabolic process [GO:0019876], xylene catabolic process [GO:0042184], toluene catabolic process [GO:0042203], s-triazine compound catabolic process [GO:0042204], halogenated hydrocarbon catabolic process [GO:0042206], GO:0042207, GO:0042208, GO:0042216, exogenous antibiotic catabolic process [GO:0042740], GO:0043421, methylnaphthalene catabolic process [GO:0043635], GO:0043636, 4-nitrophenol catabolic process [GO:0046196], GO:0046199, GO:0046213, 2-aminobenzenesulfonate catabolic process [GO:0046230], carbazole catabolic process [GO:0046232], phthalate catabolic process [GO:0046239], thiocyanate catabolic process [GO:0046265], 2-nitropropane catabolic process [GO:0046304], organosilicon catabolic process [GO:0046455], insecticide catabolic process [GO:0046701], biphenyl catabolic process [GO:0070980] Also known as: xenobiotic breakdown, xenobiotic catabolism, xenobiotic degradation, drug breakdown, drug catabolic process, drug catabolism, drug degradation, exogenous drug breakdown, exogenous drug catabolic process, exogenous drug catabolism, exogenous drug degradation